cell wall beta-glucan biosynthetic process [GO:0034410] (biological process) Subtypes: GO:0034411, plant-type cell wall cellulose biosynthetic process [GO:0052324], fungal-type cell wall beta-glucan biosynthetic process [GO:0070880] Definition: The chemical reactions and pathways resulting in the formation of beta-glucans, compounds composed of glucose residues linked by beta-D-glucosidic bonds, found in the walls of cells. Relationships: is a type of GO:0034406; is a type of beta-glucan biosynthetic process [GO:0051274]; is a type of cell wall polysaccharide biosynthetic process [GO:0070592] Also known as: cell wall beta-glucan anabolism, cell wall beta-glucan biosynthesis, cell wall beta-glucan formation, cell wall beta-glucan synthesis Sources: GOC:mah